{
  "gene_name": "Sodium-dependent phosphate transport protein 2A",
  "gene_symbol": "SLC34A1",
  "gene": "UniProtKB:Q06495",
  "term_label": "sodium:phosphate symporter activity",
  "term_id": "GO:0005436"
}